{
  "gene_symbol": "ABCF3",
  "term_label": "ATP binding",
  "gene": "UniProtKB:Q9NUQ8",
  "term_id": "GO:0005524",
  "gene_name": "ATP-binding cassette sub-family F member 3"
}